regulation of fatty acid biosynthetic process [GO:0042304] (biological process) Definition: Any process that modulates the frequency, rate or extent of the chemical reactions and pathways resulting in the formation of fatty acids, any of the aliphatic monocarboxylic acids that can be liberated by hydrolysis from naturally occurring fats and oils. Sources: GOC:go_curators, GOC:jl Also known as: regulation of fatty acid anabolism, regulation of fatty acid biosynthesis, regulation of fatty acid formation, regulation of fatty acid synthesis Relationships: is a type of GO:0019217; is a type of regulation of lipid biosynthetic process [GO:0046890]; regulates fatty acid biosynthetic process [GO:0006633] Subtypes: GO:0045717, positive regulation of fatty acid biosynthetic process [GO:0045723], regulation of jasmonic acid biosynthetic process [GO:0080141], regulation of butyryl-CoA biosynthetic process from acetyl-CoA [GO:1900494], regulation of butyryl-CoA catabolic process to butyrate [GO:1900500], regulation of methyl-branched fatty acid biosynthetic process [GO:1902322], regulation of unsaturated fatty acid biosynthetic process [GO:2001279]